D-galacturonate reductase activity [GO:0102098] (molecular function) Sources: EC:1.1.1.365, GOC:pz Relationships: is a type of oxidoreductase activity, acting on the CH-OH group of donors, NAD or NADP as acceptor [GO:0016616] Definition: Catalysis of the reaction: L-galactonate + NADP = aldehydo-D-galacturonate + NADPH + H+.